{
  "gene_symbol": "DAZ1",
  "gene_name": "Deleted in azoospermia protein 1",
  "term_label": "translation activator activity",
  "gene": "UniProtKB:Q9NQZ3",
  "term_id": "GO:0008494"
}